malonate catabolic process [GO:0090410] (biological process) Sources: GOC:tb Definition: The chemical reactions and pathways resulting in the breakdown of malonate, the propanedioate ion. Relationships: is a type of GO:0043649